{
  "gene_symbol": "EEF2",
  "gene_name": "Elongation factor 2",
  "term_id": "GO:0005829",
  "term_label": "cytosol",
  "gene": "UniProtKB:P13639"
}